maintenance of mitotic sister chromatid cohesion [GO:0034088] (biological process) Subtypes: maintenance of mitotic sister chromatid cohesion, arms [GO:0071959], maintenance of mitotic sister chromatid cohesion, centromeric [GO:0071960], maintenance of mitotic sister chromatid cohesion, telomeric [GO:0099403] Relationships: is a type of maintenance of sister chromatid cohesion [GO:0034086]; BFO_0000050 mitotic sister chromatid cohesion [GO:0007064] Sources: GOC:mah Also known as: mitotic cohesion stability Regulation: regulated by regulation of maintenance of mitotic sister chromatid cohesion [GO:0034182]; negatively regulated by GO:0034183; positively regulated by positive regulation of maintenance of mitotic sister chromatid cohesion [GO:0034184] Definition: The process in which the association between sister chromatids of a replicated chromosome is maintained as chromosomes condense, attach to the spindle in a bipolar orientation, and congress to the metaphase plate during a mitotic cell cycle.